{
  "term_label": "plasma membrane",
  "term_id": "GO:0005886",
  "gene_symbol": "TSPAN33",
  "gene_name": "Tetraspanin-33",
  "gene": "UniProtKB:Q86UF1"
}